{
  "term_label": "axon guidance",
  "gene": "UniProtKB:Q9UQ52",
  "term_id": "GO:0007411",
  "gene_symbol": "CNTN6",
  "gene_name": "Contactin-6"
}